{
  "gene": "UniProtKB:O00193",
  "term_id": "UNKNOWN:0002",
  "gene_name": "Small acidic protein",
  "gene_symbol": "SMAP",
  "term_label": "Unknown biological process"
}